{
  "term_label": "positive regulation of interleukin-5 production",
  "gene_name": "Thymic stromal lymphopoietin",
  "gene": "UniProtKB:Q969D9",
  "gene_symbol": "TSLP",
  "term_id": "GO:0032754"
}